{
  "gene_name": "Thioredoxin domain-containing protein 11",
  "gene_symbol": "TXNDC11",
  "gene": "UniProtKB:Q6PKC3",
  "term_id": "UNKNOWN:0002",
  "term_label": "Unknown biological process"
}